{
  "gene_symbol": "HAPLN1",
  "gene": "UniProtKB:P10915",
  "term_id": "GO:0005615",
  "term_label": "extracellular space",
  "gene_name": "Hyaluronan and proteoglycan link protein 1"
}